{
  "gene_symbol": "SLC22A9",
  "term_id": "GO:0015711",
  "term_label": "organic anion transport",
  "gene_name": "Organic anion transporter 7",
  "gene": "UniProtKB:Q8IVM8"
}